{
  "gene_symbol": "KCNS2",
  "term_id": "GO:0008076",
  "gene": "UniProtKB:Q9ULS6",
  "gene_name": "Potassium voltage-gated channel subfamily S member 2",
  "term_label": "voltage-gated potassium channel complex"
}